{
  "gene_symbol": "AGTR2",
  "gene": "UniProtKB:P50052",
  "term_label": "G protein-coupled receptor signaling pathway",
  "term_id": "GO:0007186",
  "gene_name": "Type-2 angiotensin II receptor"
}